{
  "gene_name": "Glycine dehydrogenase (decarboxylating), mitochondrial",
  "term_label": "glycine binding",
  "gene": "UniProtKB:P23378",
  "gene_symbol": "GLDC",
  "term_id": "GO:0016594"
}